{
  "gene": "UniProtKB:P0DTE5",
  "gene_name": "UDP-glucuronosyltransferase 2A2",
  "gene_symbol": "UGT2A2",
  "term_id": "UNKNOWN:0003",
  "term_label": "Unknown cellular component"
}